neutrophil aggregation [GO:0070488] (biological process) Relationships: is a type of leukocyte aggregation [GO:0070486] Definition: The adhesion of one neutrophil to one or more other neutrophils via adhesion molecules. Also known as: neutrocyte aggregation, neutrophil leucocyte aggregation, neutrophil leukocyte aggregation, neutrophilic leucocyte aggregation, neutrophilic leukocyte aggregation References: PMID:12972508 Sources: GOC:sl Regulation: regulated by regulation of neutrophil aggregation [GO:2000428]; negatively regulated by negative regulation of neutrophil aggregation [GO:2000429]; positively regulated by positive regulation of neutrophil aggregation [GO:2000430]